{
  "gene": "UniProtKB:Q5VYS8",
  "term_id": "UNKNOWN:0003",
  "gene_name": "Terminal uridylyltransferase 7",
  "term_label": "Unknown cellular component",
  "gene_symbol": "TUT7"
}